right anterior flagellum [GO:0097555] (cellular component) Also known as: right anterior cilium Relationships: is a type of 9+2 motile cilium [GO:0097729] Note: Note that we deem cilium and microtubule-based flagellum to be equivalent; the primary term name reflects frequency of use. Also note that, due to the asymmetric nature of the Giardia trophozoite, this term is defined spatially as the trophozoite is viewed from the dorsal side, with the two nuclei dorsal to the ventral disc, and the ventral disc toward the anterior. References: PMID:16607022, PMID:5961344 Sources: GOC:giardia, ISBN:9780124260207 Definition: A cilium (also called flagellum) found in Giardia species (trophozoite stage). It originates at the right anterior basal body, extends laterally through the cytoplasm, crosses the left anterior axoneme, and exits as a membrane-bound flagellum on the anterior right side of the cell.